symbiont-mediated suppression of host inflammatory response [GO:0052036] (biological process) Also known as: negative regulation by organism of inflammatory response of other organism involved in symbiotic interaction, down regulation by symbiont of host inflammatory response, down-regulation by symbiont of host inflammatory response, downregulation by symbiont of host inflammatory response, negative regulation by symbiont of host inflammatory response, suppression by symbiont of host inflammatory response, inhibition by symbiont of host inflammatory response Relationships: is a type of symbiont-mediated perturbation of host inflammatory response [GO:0052032] Sources: GOC:mtg_pamgo_17jul06 Definition: A process in which a symbiont inhibits or disrupts the normal execution of  inflammatory response in the host organism; the inflammatory response is the immediate defensive reaction (by vertebrate tissue) to infection or injury caused by chemical or physical agents. The host is defined as the larger of the organisms involved in a symbiotic interaction.